{
  "gene_symbol": "MRPL12",
  "term_label": "mitochondrial large ribosomal subunit",
  "gene_name": "Large ribosomal subunit protein bL12m",
  "gene": "UniProtKB:P52815",
  "term_id": "GO:0005762"
}